positive regulation of kidney development [GO:0090184] (biological process) Also known as: positive regulation of nephrogenesis Sources: GOC:dph, GOC:tb, GOC:yaf Subtypes: positive regulation of mesonephros development [GO:0061213], renal vesicle induction [GO:0072034], GO:0072216, positive regulation of metanephric cap mesenchymal cell proliferation [GO:0090096], positive regulation of glomerulus development [GO:0090193] Definition: Any process that increases the rate, frequency or extent of kidney development. Kidney development is the process whose specific outcome is the progression of the kidney over time, from its formation to the mature structure. The kidney is an organ that filters the blood and excretes the end products of body metabolism in the form of urine. Relationships: is a type of positive regulation of developmental process [GO:0051094]; is a type of positive regulation of multicellular organismal process [GO:0051240]; is a type of GO:0090183; positively regulates kidney development [GO:0001822]